GMP synthase (glutamine-hydrolyzing) activity [GO:0003922] (molecular function) Relationships: is a type of carbon-nitrogen ligase activity, with glutamine as amido-N-donor [GO:0016884]; is part of GMP biosynthetic process [GO:0006177] Sources: RHEA:11680 Definition: Catalysis of the reaction: ATP + XMP + L-glutamine + H2O = AMP + diphosphate + GMP + L-glutamate + 2H+. Also known as: GMP synthase (glutamine-hydrolysing), GMP synthetase (glutamine-hydrolysing), GMP synthetase (glutamine-hydrolyzing) activity, glutamine amidotransferase activity, guanosine 5'-monophosphate synthetase activity, guanosine monophosphate synthetase (glutamine-hydrolyzing), guanylate synthetase (glutamine-hydrolyzing), xanthosine 5'-phosphate amidotransferase activity, xanthosine-5'-phosphate:L-glutamine amido-ligase (AMP-forming)